{
  "gene_symbol": "KIF27",
  "term_id": "GO:0008017",
  "gene": "UniProtKB:Q86VH2",
  "term_label": "microtubule binding",
  "gene_name": "Kinesin-like protein KIF27"
}